{
  "gene_symbol": "HOXA4",
  "gene_name": "Homeobox protein Hox-A4",
  "term_label": "anterior/posterior pattern specification",
  "term_id": "GO:0009952",
  "gene": "UniProtKB:Q00056"
}